UFM1-modified protein reader activity [GO:0141185] (molecular function) Relationships: is a type of ubiquitin-like protein reader activity [GO:0140035] Also known as: UFM1 modified protein reader activity, UFM1-dependent protein binding References: PMID:32537488, PMID:36848233, PMID:38383785, PMID:38383789 Definition: A molecular adaptor recognizes and binds a target protein containing a UFM1 modification and brings the target protein into contact with another protein to allow those proteins to function in a coordinated way.